{
  "gene_name": "Rho GTPase-activating protein 32",
  "gene_symbol": "ARHGAP32",
  "gene": "UniProtKB:A7KAX9",
  "term_id": "GO:0098978",
  "term_label": "glutamatergic synapse"
}